{
  "term_id": "UNKNOWN:0002",
  "term_label": "Unknown biological process",
  "gene": "UniProtKB:Q7Z5Y7",
  "gene_name": "BTB_POZ domain-containing protein KCTD20",
  "gene_symbol": "KCTD20"
}